{
  "gene_symbol": "ADGRG2",
  "gene": "UniProtKB:Q8IZP9",
  "term_label": "plasma membrane",
  "term_id": "GO:0005886",
  "gene_name": "Adhesion G-protein coupled receptor G2"
}